{
  "gene_name": "POU domain, class 5, transcription factor 1",
  "term_id": "UNKNOWN:0003",
  "gene": "UniProtKB:Q01860",
  "gene_symbol": "POU5F1",
  "term_label": "Unknown cellular component"
}